uracil biosynthetic process [GO:0046107] (biological process) Subtypes: uracil salvage [GO:0006223] Sources: GOC:go_curators Relationships: is a type of GO:0019856; is a type of uracil metabolic process [GO:0019860] Definition: The chemical reactions and pathways resulting in the formation of uracil, 2,4-dioxopyrimidine, one of the pyrimidine bases occurring in RNA, but not in DNA. Also known as: uracil anabolism, uracil biosynthesis, uracil formation, uracil synthesis